{
  "gene": "UniProtKB:Q04912",
  "gene_name": "Macrophage-stimulating protein receptor",
  "term_label": "plasma membrane",
  "term_id": "GO:0005886",
  "gene_symbol": "MST1R"
}